{
  "term_id": "UNKNOWN:0002",
  "gene": "UniProtKB:Q92499",
  "gene_symbol": "DDX1",
  "term_label": "Unknown biological process",
  "gene_name": "ATP-dependent RNA helicase DDX1"
}